{
  "term_id": "UNKNOWN:0001",
  "gene_name": "Putative uncharacterized protein MSANTD5",
  "gene_symbol": "MSANTD5",
  "term_label": "Unknown molecular function",
  "gene": "UniProtKB:A0A3B3IT52"
}